{
  "term_id": "GO:0008083",
  "gene_symbol": "VEGFA",
  "term_label": "growth factor activity",
  "gene": "UniProtKB:P15692",
  "gene_name": "Vascular endothelial growth factor A, long form"
}